symbiont-mediated perturbation of host neurotransmitter secretion [GO:0044079] (biological process) Subtypes: GO:0044762 Relationships: is a type of symbiont-mediated perturbation of host cellular process [GO:0044068] Sources: MITRE:tk Definition: A process in which a symbiont alters or subverts the regulated release of a neurotransmitter from a cell in its host organism. Also known as: modification by symbiont of host neurotransmitter secretion, modulation by symbiont of host neurotransmitter secretion, modulation of host neurotransmitter secretion by symbiont, regulation by symbiont of host neurotransmitter secretion